U4/U6 snRNP [GO:0071001] (cellular component) Definition: A ribonucleoprotein complex that contains the extensively base paired small nuclear RNAs U4 and U6, a heptameric ring of Sm proteins associated with U4, the Lsm2-8 heptameric ring complex associated with U6, as well as several proteins that are unique to the U4 snRNP or U6 snRNPs, some of which remain associated with the U4/U6 snRNA both while the U4 snRNP is free or assembled into a series of spliceosomal complexes. References: PMID:14685174 Sources: GOC:krc, GOC:mah, ISBN:0879695897 Relationships: is a type of spliceosomal snRNP complex [GO:0097525]; has part U4 snRNP [GO:0005687]; has part U6 snRNP [GO:0005688]